{
  "gene": "UniProtKB:Q53H47",
  "gene_symbol": "SETMAR",
  "term_id": "GO:0003690",
  "gene_name": "Histone-lysine N-methyltransferase SETMAR",
  "term_label": "double-stranded DNA binding"
}